pteridine biosynthetic process [GO:0006728] (biological process) Definition: The chemical reactions and pathways resulting in the formation of pteridine, pyrazino(2,3-dipyrimidine), the parent structure of pterins and the pteroyl group. Sources: ISBN:0198506732 Also known as: pteridine anabolism, pteridine biosynthesis, pteridine formation, pteridine synthesis, pterin biosynthesis, pterin biosynthetic process Relationships: is a type of pteridine metabolic process [GO:0019889]; is a type of pteridine-containing compound biosynthetic process [GO:0042559]; is a type of pigment biosynthetic process [GO:0046148]